{
  "gene_symbol": "SCGB1D2",
  "gene": "UniProtKB:O95969",
  "term_label": "extracellular space",
  "gene_name": "Secretoglobin family 1D member 2",
  "term_id": "GO:0005615"
}